4-hydroxythreonine-4-phosphate dehydrogenase activity [GO:0050570] (molecular function) Relationships: is a type of oxidoreductase activity, acting on the CH-OH group of donors, NAD or NADP as acceptor [GO:0016616] Also known as: L-threonine 4-phosphate dehydrogenase activity, NAD(+)-dependent threonine 4-phosphate dehydrogenase activity, NAD+-dependent threonine 4-phosphate dehydrogenase activity Definition: Catalysis of the reaction: 4-(phosphooxy)-L-threonine + NAD+ = 3-amino-2-oxopropyl phosphate + CO2 + NADH. Sources: EC:1.1.1.262, RHEA:32275